{
  "gene": "UniProtKB:A1XBS5",
  "term_id": "GO:0060271",
  "gene_symbol": "CIBAR1",
  "term_label": "cilium assembly",
  "gene_name": "CBY1-interacting BAR domain-containing protein 1"
}